{
  "gene_symbol": "SPRYD7",
  "term_id": "UNKNOWN:0002",
  "gene": "UniProtKB:Q5W111",
  "gene_name": "SPRY domain-containing protein 7",
  "term_label": "Unknown biological process"
}